{
  "gene": "UniProtKB:Q15334",
  "gene_symbol": "LLGL1",
  "term_label": "Golgi to plasma membrane transport",
  "term_id": "GO:0006893",
  "gene_name": "Lethal(2) giant larvae protein homolog 1"
}